{
  "gene_symbol": "CPE",
  "gene": "UniProtKB:P16870",
  "term_id": "GO:0005615",
  "term_label": "extracellular space",
  "gene_name": "Carboxypeptidase E"
}